{
  "gene": "UniProtKB:Q86UB9",
  "gene_symbol": "TMEM135",
  "term_id": "UNKNOWN:0001",
  "term_label": "Unknown molecular function",
  "gene_name": "Transmembrane protein 135"
}